{
  "term_id": "GO:0005871",
  "term_label": "kinesin complex",
  "gene_symbol": "KIF21B",
  "gene_name": "Kinesin-like protein KIF21B",
  "gene": "UniProtKB:O75037"
}